{
  "term_label": "nucleus",
  "gene": "UniProtKB:P57055",
  "gene_symbol": "RIPPLY3",
  "term_id": "GO:0005634",
  "gene_name": "Protein ripply3"
}